{
  "gene_name": "Cyclic AMP-responsive element-binding protein 1",
  "term_label": "ATF4-CREB1 transcription factor complex",
  "gene": "UniProtKB:P16220",
  "gene_symbol": "CREB1",
  "term_id": "GO:1990589"
}